COP9 signalosome assembly [GO:0010387] (biological process) Definition: The aggregation, arrangement and bonding together of a set of components to form a COP9 signalosome. Relationships: is a type of GO:0065003 References: PMID:17307927 Also known as: signalosome assembly